{
  "term_label": "plasma membrane",
  "term_id": "GO:0005886",
  "gene_name": "Rho-related GTP-binding protein RhoN",
  "gene": "UniProtKB:P52198",
  "gene_symbol": "RND2"
}